agmatinase activity [GO:0008783] (molecular function) Also known as: agmatine amidinohydrolase, SpeB, agmatine ureohydrolase activity Definition: Catalysis of the reaction: agmatine + H2O = putrescine + urea. Relationships: is a type of hydrolase activity, acting on carbon-nitrogen (but not peptide) bonds, in linear amidines [GO:0016813] Sources: EC:3.5.3.11, RHEA:13929